{
  "gene_symbol": "NEU1",
  "gene": "UniProtKB:Q99519",
  "term_label": "lysosome",
  "gene_name": "Sialidase-1",
  "term_id": "GO:0005764"
}